pole cell development [GO:0007277] (BP) Sources: GOC:jid Definition: The process whose specific outcome is the progression of the pole cell over time, from its formation to the mature structure. Relationships: is a type of developmental process involved in reproduction [GO:0003006]; is a type of cell development [GO:0048468]; is part of gamete generation [GO:0007276]